{
  "gene": "UniProtKB:O15178",
  "gene_symbol": "TBXT",
  "term_id": "GO:0001707",
  "term_label": "mesoderm formation",
  "gene_name": "T-box transcription factor T"
}